{
  "gene_symbol": "TMEM30CP",
  "gene": "UniProtKB:A0ZSE6",
  "term_id": "UNKNOWN:0003",
  "gene_name": "Cell cycle control protein 50C",
  "term_label": "Unknown cellular component"
}